{
  "term_label": "Unknown molecular function",
  "gene": "UniProtKB:Q9Y6S9",
  "term_id": "UNKNOWN:0001",
  "gene_symbol": "RPS6KL1",
  "gene_name": "Ribosomal protein S6 kinase-like 1"
}